{
  "gene": "UniProtKB:O60547",
  "term_label": "'de novo' GDP-L-fucose biosynthetic process",
  "term_id": "GO:0042351",
  "gene_name": "GDP-mannose 4,6 dehydratase",
  "gene_symbol": "GMDS"
}